{
  "term_id": "GO:0070579",
  "gene": "UniProtKB:Q8NFU7",
  "term_label": "DNA 5-methylcytosine dioxygenase activity",
  "gene_name": "Methylcytosine dioxygenase TET1",
  "gene_symbol": "TET1"
}